{
  "gene_name": "Ephrin type-A receptor 8",
  "term_id": "GO:0005886",
  "gene_symbol": "EPHA8",
  "gene": "UniProtKB:P29322",
  "term_label": "plasma membrane"
}